{
  "gene_name": "TLC domain-containing protein 1",
  "term_label": "regulation of membrane lipid distribution",
  "term_id": "GO:0097035",
  "gene": "UniProtKB:Q96CP7",
  "gene_symbol": "TLCD1"
}